{
  "gene": "UniProtKB:O75830",
  "term_id": "UNKNOWN:0002",
  "gene_name": "Serpin I2",
  "term_label": "Unknown biological process",
  "gene_symbol": "SERPINI2"
}